{
  "gene": "UniProtKB:P82932",
  "gene_name": "Small ribosomal subunit protein bS6m",
  "term_label": "small ribosomal subunit rRNA binding",
  "term_id": "GO:0070181",
  "gene_symbol": "MRPS6"
}